hatching behavior [GO:0035187] (biological process) Relationships: is a type of behavior [GO:0007610]; is part of GO:0035188 References: PMID:10436051 Sources: GOC:pr Also known as: hatching behaviour Definition: The specific behavior of an organism during the emergence from an egg shell. In Drosophila for example, the larva swings its head reiteratively through a semicircular arc, using its mouth hooks to tear apart the chorion in front of it and thus free itself from within the egg shell.